{
  "gene": "UniProtKB:Q8NDP4",
  "term_label": "RNA polymerase II transcription regulatory region sequence-specific DNA binding",
  "gene_symbol": "ZNF439",
  "term_id": "GO:0000977",
  "gene_name": "Zinc finger protein 439"
}